regulation of base-excision repair [GO:1905051] (biological process) Relationships: is a type of GO:0006282; regulates GO:0006284 Subtypes: negative regulation of base-excision repair [GO:1905052], positive regulation of base-excision repair [GO:1905053] References: PMID:18973764 Sources: GOC:TermGenie, GOC:ah, GO_REF:0000058 Also known as: regulation of BER Definition: Any process that modulates the frequency, rate or extent of base-excision repair.